{
  "term_id": "GO:0005737",
  "gene_name": "Kinesin-like protein KIFC1",
  "gene": "UniProtKB:Q9BW19",
  "gene_symbol": "KIFC1",
  "term_label": "cytoplasm"
}